modified amino acid biosynthetic process [GO:0042398] (BP) Subtypes: amino-acid betaine biosynthetic process [GO:0006578], creatine biosynthetic process [GO:0006601], GO:0006659, glutathione biosynthetic process [GO:0006750], folic acid-containing compound biosynthetic process [GO:0009396], GO:0010250, pantothenate biosynthetic process [GO:0015940], peptidyl-1-thioglycine biosynthetic process from peptidyl-glycine [GO:0018173], GO:0019270, GO:0019298, 4-hydroxyproline biosynthetic process [GO:0019472], phosphagen biosynthetic process [GO:0042396], prenylcysteine biosynthetic process [GO:0046311], hydroxylysine biosynthetic process [GO:0046947], GO:0052703, pyrrolysine biosynthetic process [GO:0071524], ochratoxin A biosynthetic process [GO:1900818], GO:1901054, lincomycin biosynthetic process [GO:1901774], L-dopa biosynthetic process [GO:1903185] Sources: GOC:ai Definition: The chemical reactions and pathways resulting in the formation of compounds derived from amino acids, organic acids containing one or more amino substituents. Also known as: amino acid derivative biosynthetic process, cellular amino acid derivative anabolism, cellular amino acid derivative biosynthesis, cellular amino acid derivative biosynthetic process, cellular amino acid derivative formation, cellular amino acid derivative synthesis, cellular modified amino acid anabolism, cellular modified amino acid biosynthesis, cellular modified amino acid formation, cellular modified amino acid synthesis Relationships: is a type of modified amino acid metabolic process [GO:0006575]; is a type of GO:0009058